Golgi to plasma membrane protein transport [GO:0043001] (biological process) Regulation: regulated by regulation of Golgi to plasma membrane protein transport [GO:0042996]; negatively regulated by negative regulation of Golgi to plasma membrane protein transport [GO:0042997]; RO_0002213 by positive regulation of Golgi to plasma membrane protein transport [GO:0042998] Relationships: is a type of Golgi to plasma membrane transport [GO:0006893]; is a type of protein transport [GO:0015031]; is a type of establishment of protein localization to plasma membrane [GO:0061951]; is a type of protein localization to plasma membrane [GO:0072659] Sources: ISBN:0716731363 Definition: The directed movement of proteins from the Golgi to the plasma membrane in transport vesicles that move from the trans-Golgi network to the plasma membrane.